{
  "term_id": "GO:0004930",
  "term_label": "G protein-coupled receptor activity",
  "gene_symbol": "F2RL3",
  "gene": "UniProtKB:Q96RI0",
  "gene_name": "Proteinase-activated receptor 4"
}